{
  "gene_name": "Protein Dok-7",
  "gene_symbol": "DOK7",
  "term_id": "GO:0007528",
  "gene": "UniProtKB:Q18PE1",
  "term_label": "neuromuscular junction development"
}